{
  "gene_name": "Coiled-coil and C2 domain-containing protein 1B",
  "term_label": "DNA-binding transcription factor activity, RNA polymerase II-specific",
  "gene": "UniProtKB:Q5T0F9",
  "term_id": "GO:0000981",
  "gene_symbol": "CC2D1B"
}